{
  "gene": "UniProtKB:A0A075B6V2",
  "gene_symbol": "TRAJ21",
  "term_label": "Unknown cellular component",
  "gene_name": "T cell receptor alpha joining 21 (Fragment)",
  "term_id": "UNKNOWN:0003"
}